{
  "term_id": "UNKNOWN:0002",
  "gene_name": "Syntaxin-binding protein 6",
  "gene": "UniProtKB:Q8NFX7",
  "term_label": "Unknown biological process",
  "gene_symbol": "STXBP6"
}